right nucleus [GO:0097572] (cellular component) Definition: One of the two nuclei found in Giardia species (trophozoite stage). It is located on the right side of the cell when viewed from the dorsal side. Sources: GOC:giardia, ISBN:0-444-81258-X Note: Due to the asymmetric nature of the Giardia trophozoite, this term is defined spatially as the trophozoite is viewed from the dorsal side, with the two nuclei dorsal to the ventral disc, and the ventral disc toward the anterior. Relationships: is a type of GO:0005634